{
  "term_label": "L-leucine import across plasma membrane",
  "gene_symbol": "SLC3A2",
  "gene": "UniProtKB:P08195",
  "gene_name": "4F2 cell-surface antigen heavy chain",
  "term_id": "GO:1903801"
}